{
  "term_id": "GO:0000981",
  "gene_name": "Nuclear factor 1 C-type",
  "gene_symbol": "NFIC",
  "gene": "UniProtKB:P08651",
  "term_label": "DNA-binding transcription factor activity, RNA polymerase II-specific"
}